{
  "term_id": "GO:0005634",
  "gene": "UniProtKB:Q04724",
  "term_label": "nucleus",
  "gene_name": "Transducin-like enhancer protein 1",
  "gene_symbol": "TLE1"
}